{
  "term_label": "Unknown molecular function",
  "gene": "UniProtKB:Q6GPH6",
  "term_id": "UNKNOWN:0001",
  "gene_name": "Inositol 1,4,5-trisphosphate receptor-interacting protein-like 1",
  "gene_symbol": "ITPRIPL1"
}